{
  "term_id": "GO:0003735",
  "gene_name": "Small ribosomal subunit protein uS3",
  "term_label": "structural constituent of ribosome",
  "gene": "UniProtKB:P23396",
  "gene_symbol": "RPS3"
}